{
  "term_label": "peptide hormone binding",
  "gene_symbol": "VIPR2",
  "gene_name": "Vasoactive intestinal polypeptide receptor 2",
  "gene": "UniProtKB:P41587",
  "term_id": "GO:0017046"
}